positive regulation of Arp2/3 complex-mediated actin nucleation [GO:2000601] (biological process) Also known as: positive regulation of actin filament branch nucleation, positive regulation of branched actin filament nucleation Definition: Any process that activates or increases the frequency, rate or extent of Arp2/3 complex-mediated actin nucleation. Relationships: is a type of regulation of Arp2/3 complex-mediated actin nucleation [GO:0034315]; is a type of positive regulation of actin nucleation [GO:0051127]; positively regulates Arp2/3 complex-mediated actin nucleation [GO:0034314] References: PMID:21454476